{
  "gene_name": "Serine palmitoyltransferase 3",
  "gene": "UniProtKB:Q9NUV7",
  "term_label": "ceramide biosynthetic process",
  "term_id": "GO:0046513",
  "gene_symbol": "SPTLC3"
}